{
  "gene": "UniProtKB:Q96GF1",
  "term_id": "UNKNOWN:0003",
  "gene_name": "E3 ubiquitin-protein ligase RNF185",
  "term_label": "Unknown cellular component",
  "gene_symbol": "RNF185"
}